{
  "gene": "UniProtKB:Q13325",
  "gene_name": "Interferon-induced protein with tetratricopeptide repeats 5",
  "term_id": "GO:0003723",
  "term_label": "RNA binding",
  "gene_symbol": "IFIT5"
}